{
  "term_label": "RNA polymerase II transcription regulatory region sequence-specific DNA binding",
  "term_id": "GO:0000977",
  "gene_symbol": "STOX2",
  "gene_name": "Storkhead-box protein 2",
  "gene": "UniProtKB:Q9P2F5"
}